{
  "gene_name": "Delta-1-pyrroline-5-carboxylate dehydrogenase, mitochondrial",
  "term_label": "Unknown cellular component",
  "gene": "UniProtKB:P30038",
  "gene_symbol": "ALDH4A1",
  "term_id": "UNKNOWN:0003"
}